{
  "term_label": "negative regulation of transcription by RNA polymerase II",
  "term_id": "GO:0000122",
  "gene": "UniProtKB:Q9UBF1",
  "gene_name": "Melanoma-associated antigen C2",
  "gene_symbol": "MAGEC2"
}